sucrose induced translational repression [GO:0080149] (biological process) Definition: Any process that stops, prevents or reduces the rate of translation as a result of increase in sucrose level. Relationships: is a type of GO:0032055 References: PMID:19403731 Also known as: negative regulation of translation in response to sucrose